{
  "gene_symbol": "LRP1B",
  "gene": "UniProtKB:Q9NZR2",
  "term_id": "GO:0005041",
  "term_label": "low-density lipoprotein particle receptor activity",
  "gene_name": "Low-density lipoprotein receptor-related protein 1B"
}